{
  "gene_symbol": "ABCG8",
  "term_id": "GO:0042626",
  "gene_name": "ATP-binding cassette sub-family G member 8",
  "term_label": "ATPase-coupled transmembrane transporter activity",
  "gene": "UniProtKB:Q9H221"
}